{
  "term_label": "ATP hydrolysis activity",
  "gene_name": "Endoplasmic reticulum chaperone BiP",
  "gene_symbol": "HSPA5",
  "gene": "UniProtKB:P11021",
  "term_id": "GO:0016887"
}